{
  "gene": "UniProtKB:P54821",
  "gene_name": "Paired mesoderm homeobox protein 1",
  "term_id": "GO:0006357",
  "gene_symbol": "PRRX1",
  "term_label": "regulation of transcription by RNA polymerase II"
}